myelination of anterior lateral line nerve axons [GO:0048914] (biological process) Definition: The formation of compact myelin sheaths around the axons of the anterior lateral line nerve. References: PMID:12112375 Relationships: is a type of myelination of lateral line nerve axons [GO:0048897]; is part of anterior lateral line nerve glial cell morphogenesis involved in differentiation [GO:0048940]